toll-like receptor 21 signaling pathway [GO:0035682] (biological process) Regulation: regulated by GO:2000443; RO_0002212 by negative regulation of toll-like receptor 21 signaling pathway [GO:2000444]; positively regulated by GO:2000445 Also known as: TLR21 signaling pathway, toll-like receptor 21 signalling pathway Sources: GOC:pde Relationships: is a type of toll-like receptor signaling pathway [GO:0002224] Definition: The series of molecular signals initiated by a ligand binding to toll-like receptor 21.